{
  "term_id": "GO:0019905",
  "term_label": "syntaxin binding",
  "gene_name": "Synaptosomal-associated protein 23",
  "gene_symbol": "SNAP23",
  "gene": "UniProtKB:O00161"
}